{
  "term_id": "GO:0005794",
  "gene_symbol": "TANGO2",
  "gene_name": "Transport and Golgi organization protein 2 homolog",
  "gene": "UniProtKB:Q6ICL3",
  "term_label": "Golgi apparatus"
}